N-terminal peptidyl-aspartic acid acetylation [GO:0017190] (biological process) Sources: RESID:AA0042 Relationships: is_a N-terminal protein amino acid acetylation [GO:0006474]; is a type of peptidyl-aspartic acid modification [GO:0018197] Note: See also the molecular function term 'aspartate N-acetyltransferase activity ; GO:0017188'. Definition: The acetylation of the N-terminal aspartic acid of proteins; catalyzed by aspartate N-acetyltransferase.